{
  "gene_name": "Outer dense fiber protein 2",
  "term_id": "GO:1902017",
  "gene_symbol": "ODF2",
  "gene": "UniProtKB:Q5BJF6",
  "term_label": "regulation of cilium assembly"
}